atrioventricular valve development [GO:0003171] (biological process) Also known as: AV valve development Definition: The progression of the atrioventricular valve over time, from its formation to the mature structure. Relationships: is a type of GO:0003170 Subtypes: mitral valve development [GO:0003174], tricuspid valve development [GO:0003175] Sources: GOC:mtg_heart